{
  "term_id": "UNKNOWN:0003",
  "gene": "UniProtKB:Q13976",
  "gene_symbol": "PRKG1",
  "term_label": "Unknown cellular component",
  "gene_name": "cGMP-dependent protein kinase 1"
}